{
  "gene_symbol": "TUBE1",
  "gene_name": "Tubulin epsilon chain",
  "term_id": "GO:0000278",
  "gene": "UniProtKB:Q9UJT0",
  "term_label": "mitotic cell cycle"
}